{
  "term_label": "plasma membrane",
  "gene_symbol": "FRMD6",
  "gene": "UniProtKB:Q96NE9",
  "term_id": "GO:0005886",
  "gene_name": "FERM domain-containing protein 6"
}